{
  "gene_name": "Myosin light chain kinase, smooth muscle",
  "term_label": "myosin light chain kinase activity",
  "gene_symbol": "MYLK",
  "gene": "UniProtKB:Q15746",
  "term_id": "GO:0004687"
}